{
  "gene": "UniProtKB:P0C862",
  "term_label": "Unknown cellular component",
  "term_id": "UNKNOWN:0003",
  "gene_symbol": "C1QTNF9",
  "gene_name": "Complement C1q and tumor necrosis factor-related protein 9A"
}